{
  "gene_name": "Guanine nucleotide-binding protein G(z) subunit alpha",
  "term_label": "G protein-coupled receptor binding",
  "term_id": "GO:0001664",
  "gene": "UniProtKB:P19086",
  "gene_symbol": "GNAZ"
}